{
  "term_id": "GO:0005768",
  "term_label": "endosome",
  "gene": "UniProtKB:Q9UBQ0",
  "gene_symbol": "VPS29",
  "gene_name": "Vacuolar protein sorting-associated protein 29"
}